{
  "term_label": "GTP binding",
  "gene_name": "ADP-ribosylation factor 5",
  "gene_symbol": "ARF5",
  "term_id": "GO:0005525",
  "gene": "UniProtKB:P84085"
}